Photinus-luciferin 4-monooxygenase (ATP-hydrolyzing) activity [GO:0047077] (molecular function) Definition: Catalysis of the reaction: O2 + ATP + Photinus luciferin = light + diphosphate + AMP + CO2 + oxidized Photinus luciferin. Also known as: luciferase activity, Photinus luciferin 4-monooxygenase (adenosine triphosphate-hydrolyzing), Photinus pyralis luciferase activity, Photinus-luciferin 4-monooxygenase (ATP-hydrolysing), Photinus-luciferin:oxygen 4-oxidoreductase (decarboxylating, ATP-hydrolysing), firefly luciferase activity, firefly luciferin luciferase activity, luciferase (firefly luciferin) Sources: EC:1.13.12.7, MetaCyc:1.13.12.7-RXN Relationships: is a type of oxidoreductase activity, acting on single donors with incorporation of molecular oxygen, incorporation of one atom of oxygen (internal monooxygenases or internal mixed function oxidases) [GO:0016703]; is a type of luciferin monooxygenase activity [GO:0045289]